{
  "gene_name": "Histone H1.3",
  "gene": "UniProtKB:P16402",
  "term_label": "double-stranded DNA binding",
  "term_id": "GO:0003690",
  "gene_symbol": "H1-3"
}